{
  "gene_symbol": "TMED3",
  "term_label": "intracellular protein transport",
  "gene_name": "Transmembrane emp24 domain-containing protein 3",
  "term_id": "GO:0006886",
  "gene": "UniProtKB:Q9Y3Q3"
}